{
  "gene_symbol": "RPAIN",
  "term_label": "nucleus",
  "term_id": "GO:0005634",
  "gene": "UniProtKB:Q86UA6",
  "gene_name": "RPA-interacting protein"
}